{
  "gene_symbol": "TRIM51G",
  "gene_name": "Putative tripartite motif-containing protein 51G",
  "term_label": "cytoplasm",
  "gene": "UniProtKB:A0A3B3IT33",
  "term_id": "GO:0005737"
}